regulation of embryonic development [GO:0045995] (biological process) Relationships: is a type of regulation of multicellular organismal development [GO:2000026]; regulates embryo development [GO:0009790] Sources: GOC:go_curators Definition: Any process that modulates the frequency, rate or extent of embryonic development. Subtypes: inhibition of neuroepithelial cell differentiation [GO:0002085], GO:0010470, regulation of embryonic cell shape [GO:0016476], positive regulation of embryonic development [GO:0040019], GO:0045992, lung induction [GO:0060492], GO:0060787, regulation of basement membrane assembly involved in embryonic body morphogenesis [GO:1904259]